cyanelle thylakoid membrane [GO:0033115] (cellular component) Sources: GOC:mah Definition: The lipid bilayer membrane of any thylakoid within a cyanelle. Relationships: is a type of plastid thylakoid membrane [GO:0055035]; is part of cyanelle thylakoid [GO:0009843]